endosome transport via multivesicular body sorting pathway [GO:0032509] (biological process) Definition: The directed movement of substances from endosomes to lysosomes or vacuoles by a pathway in which molecules are sorted into multivesicular bodies, which then fuse with the target compartment. References: PMID:12461556, PMID:16689637 Sources: GOC:mah Also known as: endosome transport via MVB sorting pathway Relationships: is a type of endosomal transport [GO:0016197]; is a type of multivesicular body sorting pathway [GO:0071985] Subtypes: endosome to lysosome transport via multivesicular body sorting pathway [GO:0032510], late endosome to vacuole transport via multivesicular body sorting pathway [GO:0032511]